{
  "gene_name": "Protein inscuteable homolog",
  "term_label": "cytoskeletal anchor activity",
  "gene_symbol": "INSC",
  "term_id": "GO:0008093",
  "gene": "UniProtKB:Q1MX18"
}